{
  "term_label": "Rap protein signal transduction",
  "gene_name": "Rap guanine nucleotide exchange factor 6",
  "gene_symbol": "RAPGEF6",
  "gene": "UniProtKB:Q8TEU7",
  "term_id": "GO:0032486"
}